{
  "term_id": "GO:0035036",
  "gene_symbol": "SPACA4",
  "gene": "UniProtKB:Q8TDM5",
  "gene_name": "Sperm acrosome membrane-associated protein 4",
  "term_label": "sperm-egg recognition"
}